{
  "term_id": "UNKNOWN:0002",
  "gene": "UniProtKB:Q16774",
  "gene_name": "Guanylate kinase",
  "term_label": "Unknown biological process",
  "gene_symbol": "GUK1"
}